{
  "gene": "UniProtKB:P62942",
  "gene_name": "Peptidyl-prolyl cis-trans isomerase FKBP1A",
  "term_label": "peptidyl-prolyl cis-trans isomerase activity",
  "term_id": "GO:0003755",
  "gene_symbol": "FKBP1A"
}